{
  "term_id": "GO:0015245",
  "gene": "UniProtKB:Q8NA29",
  "gene_name": "Sodium-dependent lysophosphatidylcholine symporter 1",
  "gene_symbol": "MFSD2A",
  "term_label": "fatty acid transmembrane transporter activity"
}